mesenchymal to epithelial transition involved in metanephric renal vesicle formation [GO:0072285] (biological process) Definition: A transition where a mesenchymal cell establishes apical/basolateral polarity,forms intercellular adhesive junctions, synthesizes basement membrane components and becomes an epithelial cell that will contribute to the shaping of the metanephric renal vesicle. Sources: GOC:mtg_kidney_jan10 Relationships: is a type of mesenchymal to epithelial transition involved in metanephros morphogenesis [GO:0003337]; is a type of GO:0072036; BFO_0000050 metanephric renal vesicle formation [GO:0072093]